glycoRNA biosynthetic process [GO:0141217] (biological process) Definition: The posttranscriptional addition of a carbohydrate or carbohydrate derivative unit to residues in an RNA molecule. GlycoRNA consists of RNAs modified with secretory N-glycans that are presented on the cell surface. References: PMID:34004145, PMID:39173631 Relationships: is a type of GO:0006396 Also known as: RNA glycosylation, glycoRNA biosynthesis